cellular response to cell envelope stress [GO:0036460] (biological process) Relationships: is_a cellular response to stress [GO:0033554] Definition: Any process that results in a change in state or activity of a cell (in terms of movement, secretion, enzyme production, gene expression, etc.) as a result of stress acting at the cell envelope. Also known as: envelope stress response References: PMID:15101969, PMID:15882407 Sources: GOC:imk